{
  "term_label": "ATP hydrolysis activity",
  "term_id": "GO:0016887",
  "gene_symbol": "KIF7",
  "gene": "UniProtKB:Q2M1P5",
  "gene_name": "Kinesin-like protein KIF7"
}